regulation of infection cushion formation [GO:0075184] (biological process) Subtypes: GO:0075185, negative regulation of infection cushion formation [GO:0075186] Also known as: regulation of infection cushion formation on or near host Relationships: is a type of regulation of developmental process [GO:0050793]; regulates infection cushion formation [GO:0075183] Sources: GOC:pamgo_curators Definition: Any process that modulates the frequency, rate or extent of symbiont infection cushion formation.